{
  "gene": "UniProtKB:P47869",
  "gene_name": "Gamma-aminobutyric acid receptor subunit alpha-2",
  "term_label": "synaptic transmission, GABAergic",
  "term_id": "GO:0051932",
  "gene_symbol": "GABRA2"
}